{
  "term_label": "cytoplasm",
  "gene_symbol": "TRIM73",
  "gene_name": "Tripartite motif-containing protein 73",
  "term_id": "GO:0005737",
  "gene": "UniProtKB:Q86UV7"
}